{
  "gene_name": "Endophilin-A3",
  "gene": "UniProtKB:Q99963",
  "term_label": "protein-macromolecule adaptor activity",
  "term_id": "GO:0030674",
  "gene_symbol": "SH3GL3"
}